{
  "term_label": "heterochromatin formation",
  "term_id": "GO:0031507",
  "gene": "UniProtKB:Q9BTM1",
  "gene_symbol": "H2AJ",
  "gene_name": "Histone H2A.J"
}